positive regulation of snoRNA metabolic process [GO:1903325] (biological process) Definition: Any process that activates or increases the frequency, rate or extent of snoRNA metabolic process. Also known as: positive regulation of snoRNA metabolism, up regulation of snoRNA metabolic process, up regulation of snoRNA metabolism, up-regulation of snoRNA metabolic process, up-regulation of snoRNA metabolism, upregulation of snoRNA metabolic process, upregulation of snoRNA metabolism, activation of snoRNA metabolic process, activation of snoRNA metabolism Sources: GOC:TermGenie, GOC:vw, GO_REF:0000058 Subtypes: positive regulation of snoRNA processing [GO:1902798] Relationships: is a type of positive regulation of RNA metabolic process [GO:0051254]; is a type of GO:1903323; RO_0002213 sno(s)RNA metabolic process [GO:0016074]